{
  "term_id": "GO:0005912",
  "gene": "UniProtKB:Q9UJ99",
  "gene_name": "Cadherin-22",
  "term_label": "adherens junction",
  "gene_symbol": "CDH22"
}